{
  "term_label": "regulation of transcription by RNA polymerase II",
  "gene": "UniProtKB:Q96PT4",
  "gene_symbol": "DUX3",
  "term_id": "GO:0006357",
  "gene_name": "Putative double homeobox protein 3"
}